{
  "term_label": "intracellular signal transduction",
  "gene_name": "SH3 domain-binding protein 5-like",
  "term_id": "GO:0035556",
  "gene": "UniProtKB:Q7L8J4",
  "gene_symbol": "SH3BP5L"
}